flavin-dependent halogenase activity [GO:0140907] (molecular function) Definition: Catalysis of the reaction: R-CH + a halogen + FADH2 + O2 = R-C-halogen + FAD + H2O. References: PMID:28466644, PMID:34368824 Relationships: is a type of halogenase activity [GO:0140906]